{
  "term_id": "GO:0003779",
  "gene_name": "Microtubule-associated protein 1B",
  "term_label": "actin binding",
  "gene_symbol": "MAP1B",
  "gene": "UniProtKB:P46821"
}